{
  "gene": "UniProtKB:A6NF01",
  "term_label": "RNA export from nucleus",
  "gene_name": "Putative nuclear envelope pore membrane protein POM 121B",
  "gene_symbol": "POM121B",
  "term_id": "GO:0006405"
}